glomus development [GO:0072013] (BP) Relationships: is a type of anatomical structure development [GO:0048856]; is part of pronephros development [GO:0048793] Also known as: pronephric glomus development References: PMID:10572058, PMID:15647339, PMID:9268568 Sources: GOC:mtg_kidney_jan10, XAO:0000318 Definition: The progression of the glomus over time from its initial formation until its mature state. The glomus forms from the splanchnic intermediate mesoderm and is the vascularized filtration unit, filtering the blood before it enters the tubules. The glomus is external to the nephron and extends over more than one body segment.